{
  "term_label": "maintenance of gastrointestinal epithelium",
  "gene_symbol": "VSIG1",
  "gene_name": "V-set and immunoglobulin domain-containing protein 1",
  "gene": "UniProtKB:Q86XK7",
  "term_id": "GO:0030277"
}